{
  "gene_symbol": "P4HA3",
  "term_label": "collagen fibril organization",
  "gene": "UniProtKB:Q7Z4N8",
  "term_id": "GO:0030199",
  "gene_name": "Prolyl 4-hydroxylase subunit alpha-3"
}